{
  "gene_name": "Homeobox protein VENTX",
  "gene": "UniProtKB:O95231",
  "gene_symbol": "VENTX",
  "term_label": "regulation of transcription by RNA polymerase II",
  "term_id": "GO:0006357"
}